{
  "term_label": "Prp19 complex",
  "gene_name": "Pre-mRNA-splicing factor SYF2",
  "gene_symbol": "SYF2",
  "term_id": "GO:0000974",
  "gene": "UniProtKB:O95926"
}